{
  "term_label": "all-trans-retinol dehydrogenase (NAD+) activity",
  "gene_name": "Short-chain dehydrogenase_reductase family 9C member 7",
  "term_id": "GO:0004745",
  "gene_symbol": "SDR9C7",
  "gene": "UniProtKB:Q8NEX9"
}